{
  "term_id": "GO:0005886",
  "gene": "UniProtKB:Q9NRQ2",
  "gene_name": "Phospholipid scramblase 4",
  "gene_symbol": "PLSCR4",
  "term_label": "plasma membrane"
}